{
  "gene_symbol": "HTR1B",
  "term_label": "plasma membrane",
  "term_id": "GO:0005886",
  "gene_name": "5-hydroxytryptamine receptor 1B",
  "gene": "UniProtKB:P28222"
}